pigment accumulation in tissues in response to UV light [GO:0043479] (biological process) Subtypes: anthocyanin accumulation in tissues in response to UV light [GO:0043481] Sources: GOC:jl Relationships: is_a pigment accumulation in response to UV light [GO:0043478]; is a type of GO:0043480 Definition: The aggregation of coloring matter in a particular location in a tissue, occurring in response to a UV light stimulus.